positive regulation of ovulation [GO:0060279] (biological process) Definition: Any process that activates or increases the frequency, rate or extent of ovulation, the release of a mature ovum/oocyte from an ovary. Sources: GOC:dph, GOC:kmv, GOC:tb Relationships: is a type of GO:0051240; is_a regulation of ovulation [GO:0060278]; is a type of GO:2000243; positively regulates GO:0030728